{
  "term_label": "retinoic acid metabolic process",
  "gene_symbol": "ADH6",
  "term_id": "GO:0042573",
  "gene": "UniProtKB:P28332",
  "gene_name": "Alcohol dehydrogenase 6"
}